positive regulation of calcium ion import [GO:0090280] (biological process) Sources: GOC:BHF Definition: Any process that increases the rate, frequency, or extent of the directed movement of calcium ions into a cell or organelle. Also known as: positive regulation of transmembrane calcium influx Subtypes: positive regulation of calcium ion import across plasma membrane [GO:1905665] Relationships: is a type of positive regulation of calcium ion transport [GO:0051928]; is a type of regulation of calcium ion import [GO:0090279]; positively regulates GO:0070509